renal system process involved in regulation of systemic arterial blood pressure [GO:0003071] (biological process) Also known as: renal control of blood pressure, renal regulation of systemic arterial blood pressure Definition: Renal process that modulates the force with which blood travels through the circulatory system. The process is controlled by a balance of processes that increase pressure and decrease pressure. Relationships: is_a renal system process [GO:0003014]; is part of regulation of systemic arterial blood pressure [GO:0003073] Subtypes: GO:0001977, renal response to blood flow involved in circulatory renin-angiotensin regulation of systemic arterial blood pressure [GO:0001999], renin-angiotensin regulation of aldosterone production [GO:0002018], GO:0003072 Sources: GOC:dph, GOC:mtg_cardio, GOC:tb